{
  "gene_symbol": "HMX2",
  "gene": "UniProtKB:A2RU54",
  "term_id": "GO:0000977",
  "gene_name": "Homeobox protein HMX2",
  "term_label": "RNA polymerase II transcription regulatory region sequence-specific DNA binding"
}